positive regulation of mitochondrial RNA catabolic process [GO:0000962] (biological process) Subtypes: positive regulation of mitochondrial mRNA catabolic process [GO:1905639] Sources: GOC:krc, GOC:mah Definition: Any process that activates or increases the frequency, rate or extent of the chemical reactions and pathways involving catabolism in the mitochondrion of RNA transcribed from the mitochondrial genome. Relationships: is a type of regulation of mitochondrial RNA catabolic process [GO:0000960]; is a type of positive regulation of catabolic process [GO:0009896]; is a type of positive regulation of RNA metabolic process [GO:0051254]; positively regulates GO:0000957